{
  "gene_symbol": "FGF7",
  "gene_name": "Fibroblast growth factor 7",
  "gene": "UniProtKB:P21781",
  "term_id": "GO:0005111",
  "term_label": "type 2 fibroblast growth factor receptor binding"
}